histone H3K14 ubiquitin ligase activity [GO:0140851] (molecular function) Definition: Catalysis of the transfer of a ubiquitin molecule to histone 3 at the lysine-14 residue. References: PMID:28624371, PMID:31468675, PMID:34010645 Also known as: histone H3-K14 ubiquitin ligase activity, histone ubiquitin ligase activity (H3-K14 specific) Note: Comment: Note that the residue position corresponds to the canonical human H3 histone (UniProtKB:P84243); this residue is conserved across all eukaryotes. Residue 1 is the first residue following removal of the initiating Methionine (Met). Note that each histone is encoded by multiple genes, and sequences may vary across different genes within an organism. Relationships: is a type of histone H3 ubiquitin ligase activity [GO:0141055]